protein tyrosine phosphatase activity [GO:0004725] (molecular function) Regulation: positively regulated by protein tyrosine phosphatase activator activity [GO:0008160] Sources: EC:3.1.3.48 Definition: Catalysis of the reaction: protein tyrosine phosphate + H2O = protein tyrosine + phosphate. Also known as: PPT-phosphatase activity, PTP-phosphatase activity, PTPase activity, [phosphotyrosine]protein phosphatase activity, phosphoprotein phosphatase (phosphotyrosine) activity, phosphotyrosine histone phosphatase activity, phosphotyrosine phosphatase activity, phosphotyrosine protein phosphatase activity, phosphotyrosylprotein phosphatase activity, protein phosphotyrosine phosphatase activity, protein-tyrosine-phosphatase activity, protein-tyrosine-phosphate phosphohydrolase activity, tyrosine O-phosphate phosphatase activity, tyrosylprotein phosphatase activity Relationships: is a type of phosphoprotein phosphatase activity [GO:0004721] Subtypes: non-membrane spanning protein tyrosine phosphatase activity [GO:0004726], transmembrane receptor protein tyrosine phosphatase activity [GO:0005001], GO:0030946, GO:0033550